{
  "gene": "UniProtKB:Q99435",
  "gene_name": "Protein kinase C-binding protein NELL2",
  "gene_symbol": "NELL2",
  "term_id": "GO:0005737",
  "term_label": "cytoplasm"
}